{
  "gene_symbol": "PKP3",
  "term_id": "GO:0005634",
  "term_label": "nucleus",
  "gene_name": "Plakophilin-3",
  "gene": "UniProtKB:Q9Y446"
}